uronic acid transmembrane transport [GO:0015735] (biological process) Subtypes: hexuronate transmembrane transport [GO:0015736] Relationships: is_a monocarboxylic acid transport [GO:0015718]; is a type of carboxylic acid transmembrane transport [GO:1905039] Sources: GOC:krc Definition: The process in which uronic acid is transported across a lipid bilayer, from one side of a membrane to the other. Also known as: uronic acid transport